{
  "gene": "UniProtKB:P61769",
  "term_label": "late endosome membrane",
  "term_id": "GO:0031902",
  "gene_name": "Beta-2-microglobulin",
  "gene_symbol": "B2M"
}